{
  "gene_name": "Osteocalcin",
  "gene": "UniProtKB:P02818",
  "term_id": "GO:0060348",
  "gene_symbol": "BGLAP",
  "term_label": "bone development"
}